{
  "gene_name": "Peroxisomal sarcosine oxidase",
  "term_id": "GO:0050031",
  "gene_symbol": "PIPOX",
  "term_label": "L-pipecolate oxidase activity",
  "gene": "UniProtKB:Q9P0Z9"
}